{
  "gene_name": "Pleckstrin homology domain-containing family A member 3",
  "term_label": "early endosome",
  "gene": "UniProtKB:Q9HB20",
  "gene_symbol": "PLEKHA3",
  "term_id": "GO:0005769"
}